branching morphogenesis of a nerve [GO:0048755] (biological process) Relationships: is a type of morphogenesis of a branching structure [GO:0001763]; is part of nervous system development [GO:0007399] Definition: The process in which the anatomical structures of branches in a nerve are generated and organized. This term refers to an anatomical structure (nerve) not a cell (neuron). Regulation: positively regulated by positive regulation of branching morphogenesis of a nerve [GO:1905492]; regulated by regulation of branching morphogenesis of a nerve [GO:2000172]; negatively regulated by negative regulation of branching morphogenesis of a nerve [GO:2000173] Sources: GOC:dgh, GOC:dph, GOC:jid